{
  "term_label": "mitochondrion",
  "gene_name": "Cytochrome c oxidase assembly factor 6 homolog",
  "gene": "UniProtKB:Q5JTJ3",
  "gene_symbol": "COA6",
  "term_id": "GO:0005739"
}